phosphoglucosamine mutase activity [GO:0008966] (molecular function) Also known as: D-glucosamine 1,6-phosphomutase activity, alpha-D-glucosamine 1,6-phosphomutase activity Definition: Catalysis of the reaction: alpha-D-glucosamine 1-phosphate = D-glucosamine 6-phosphate. Sources: EC:5.4.2.10, RHEA:23424 Relationships: is a type of intramolecular phosphotransferase activity [GO:0016868]